keratan sulfotransferase activity [GO:0045130] (molecular function) Definition: Catalysis of the reaction: 3'-phosphoadenosine 5'-phosphosulfate + keratan = adenosine 3',5'-bisphosphate + keratan 6'-sulfate. Sources: EC:2.8.2.21 Also known as: keratan sulfate Gal-6-sulfotransferase activity, keratan sulphotransferase activity, 3'-phosphoadenylyl keratan sulfotransferase activity, 3'-phosphoadenylyl-sulfate:keratan 6'-sulfotransferase activity, 3'-phosphoadenylylsulfate:keratan sulfotransferase activity, keratan sulfate sulfotransferase activity Relationships: is a type of proteoglycan sulfotransferase activity [GO:0050698]